{
  "gene_name": "Charged multivesicular body protein 4c",
  "gene": "UniProtKB:Q96CF2",
  "term_label": "cytoplasmic side of plasma membrane",
  "term_id": "GO:0009898",
  "gene_symbol": "CHMP4C"
}